{
  "gene_name": "Myelin P2 protein",
  "term_label": "nucleus",
  "term_id": "GO:0005634",
  "gene_symbol": "PMP2",
  "gene": "UniProtKB:P02689"
}